{
  "term_id": "UNKNOWN:0001",
  "gene": "UniProtKB:C9JC47",
  "gene_name": "Putative protein FAM157A",
  "gene_symbol": "FAM157A",
  "term_label": "Unknown molecular function"
}